{
  "gene_name": "Cdc42 effector protein 5",
  "term_id": "GO:0005856",
  "gene_symbol": "CDC42EP5",
  "gene": "UniProtKB:Q6NZY7",
  "term_label": "cytoskeleton"
}